{
  "gene_name": "DNA polymerase delta subunit 4",
  "gene": "UniProtKB:Q9HCU8",
  "gene_symbol": "POLD4",
  "term_label": "DNA synthesis involved in DNA repair",
  "term_id": "GO:0000731"
}